{
  "term_label": "branched-chain amino acid transmembrane transporter activity",
  "gene_name": "Solute carrier family 25 member 44",
  "term_id": "GO:0015658",
  "gene": "UniProtKB:Q96H78",
  "gene_symbol": "SLC25A44"
}